structural constituent of pupal chitin-based cuticle [GO:0008011] (molecular function) Relationships: is a type of structural constituent of chitin-based cuticle [GO:0005214] Sources: GOC:mah, GOC:mtg_sensu Definition: The action of a molecule that contributes to the structural integrity of the chitin-based cuticle of a pupa. An example of this is found in Drosophila melanogaster. Also known as: structural constituent of pupal cuticle